{
  "gene_name": "Histone-lysine N-methyltransferase PRDM9",
  "term_label": "recombination hotspot binding",
  "gene": "UniProtKB:Q9NQV7",
  "term_id": "GO:0010844",
  "gene_symbol": "PRDM9"
}